{
  "term_id": "UNKNOWN:0001",
  "gene_symbol": "C2orf78",
  "term_label": "Unknown molecular function",
  "gene_name": "Uncharacterized protein C2orf78",
  "gene": "UniProtKB:A6NCI8"
}